retrotrapezoid nucleus neuron differentiation [GO:0061452] (biological process) Relationships: is a type of central nervous system neuron differentiation [GO:0021953]; is part of retrotrapezoid nucleus development [GO:0061451] Definition: The process in which a relatively unspecialized cell acquires specialized features of a neuron whose cell body resides in the retrotrapezoid nucleus. Sources: GOC:dph